{
  "term_id": "GO:0001518",
  "gene": "UniProtKB:O60939",
  "gene_name": "Sodium channel subunit beta-2",
  "gene_symbol": "SCN2B",
  "term_label": "voltage-gated sodium channel complex"
}